{
  "gene_symbol": "GALNT15",
  "term_label": "Golgi apparatus",
  "term_id": "GO:0005794",
  "gene_name": "Polypeptide N-acetylgalactosaminyltransferase 15",
  "gene": "UniProtKB:Q8N3T1"
}